{
  "gene_symbol": "CDK17",
  "term_label": "nucleus",
  "gene": "UniProtKB:Q00537",
  "term_id": "GO:0005634",
  "gene_name": "Cyclin-dependent kinase 17"
}